{
  "term_id": "GO:0005634",
  "term_label": "nucleus",
  "gene_name": "Telomere-associated protein RIF1",
  "gene_symbol": "RIF1",
  "gene": "UniProtKB:Q5UIP0"
}